{
  "gene_symbol": "RAET1E",
  "gene": "UniProtKB:Q8TD07",
  "term_id": "GO:0048018",
  "gene_name": "Retinoic acid early transcript 1E",
  "term_label": "receptor ligand activity"
}